{
  "gene_symbol": "OR5AP2",
  "term_label": "olfactory receptor activity",
  "gene": "UniProtKB:Q8NGF4",
  "gene_name": "Olfactory receptor 5AP2",
  "term_id": "GO:0004984"
}